negative regulation of hemicellulose catabolic process [GO:2000989] (biological process) Subtypes: negative regulation of xyloglucan catabolic process [GO:2000952], GO:2001001 Also known as: negative regulation of hemicellulose catabolism Definition: Any process that stops, prevents or reduces the frequency, rate or extent of hemicellulose catabolic process. Relationships: is a type of negative regulation of catabolic process [GO:0009895]; is a type of negative regulation of macromolecule metabolic process [GO:0010605]; is_a negative regulation of carbohydrate metabolic process [GO:0045912]; is a type of regulation of hemicellulose catabolic process [GO:2000988]; negatively regulates hemicellulose catabolic process [GO:2000895] Sources: GOC:mengo_curators